myo-inositol:proton symporter activity [GO:0005366] (molecular function) Sources: TC:2.A.1.1.8 Relationships: is a type of myo-inositol transmembrane transporter activity [GO:0005365]; is a type of solute:proton symporter activity [GO:0015295] Also known as: hydrogen/myo-inositol transporter activity, myo-inositol:hydrogen symporter activity Definition: Enables the transfer of a solute or solutes from one side of a membrane to the other according to the reaction: myo-inositol(out) + H+(out) = myo-inositol(in) + H+(in).